{
  "term_label": "adenylate cyclase-activating G protein-coupled receptor signaling pathway",
  "gene_symbol": "GPR157",
  "gene_name": "G-protein coupled receptor 157",
  "gene": "UniProtKB:Q5UAW9",
  "term_id": "GO:0007189"
}